{
  "term_label": "regulation of organelle assembly",
  "gene_symbol": "RDX",
  "gene": "UniProtKB:P35241",
  "term_id": "GO:1902115",
  "gene_name": "Radixin"
}